{
  "term_label": "cell motility",
  "term_id": "GO:0048870",
  "gene": "UniProtKB:Q96BJ8",
  "gene_name": "Engulfment and cell motility protein 3",
  "gene_symbol": "ELMO3"
}